{
  "term_label": "GTPase activity",
  "gene_symbol": "MTG1",
  "term_id": "GO:0003924",
  "gene": "UniProtKB:Q9BT17",
  "gene_name": "Mitochondrial ribosome-associated GTPase 1"
}